negative regulation of phosphatidylinositol 3-kinase/protein kinase B signal transduction [GO:0051898] (biological process) Sources: GOC:ai Definition: Any process that stops, prevents, or reduces the frequency, rate or extent of phosphatidylinositol 3-kinase/protein kinase B signal transduction. Also known as: negative regulation of PI3K-PKB/Akt pathway, negative regulation of PI3K/Akt signal transduction, negative regulation of PI3K/PKB signal transduction, negative regulation of phosphatidylinositol 3-kinase signaling/protein kinase B signal transduction, inhibition of protein kinase B signaling cascade, down regulation of protein kinase B signaling cascade, down-regulation of protein kinase B signaling cascade, downregulation of protein kinase B signaling cascade, negative regulation of AKT signaling cascade, negative regulation of AKT signalling cascade, negative regulation of PKB signaling cascade, negative regulation of PKB signalling cascade, negative regulation of protein kinase B signaling, negative regulation of protein kinase B signaling cascade, negative regulation of protein kinase B signalling cascade Relationships: is a type of GO:0051896; is a type of negative regulation of intracellular signal transduction [GO:1902532]; negatively regulates phosphatidylinositol 3-kinase/protein kinase B signal transduction [GO:0043491]